{
  "gene_symbol": "PIK3CA",
  "gene": "UniProtKB:P42336",
  "term_label": "phosphatidylinositol-mediated signaling",
  "term_id": "GO:0048015",
  "gene_name": "Phosphatidylinositol 4,5-bisphosphate 3-kinase catalytic subunit alpha isoform"
}